UFM1 transferase activity [GO:0071568] (MF) Subtypes: UFM1 conjugating enzyme activity [GO:0061657], UFM1 ligase activity [GO:0061666] Relationships: is a type of GO:0019787 Definition: Catalysis of the transfer of UFM1 from one protein to another via the reaction X-UFM1 + Y = Y-UFM1 + X, where both X-UFM1 and Y-UFM1 are covalent linkages. References: PMID:20018847 Sources: GOC:sp